establishment of spindle localization [GO:0051293] (biological process) Definition: The directed movement of the spindle to a specific location in the cell. Relationships: is a type of GO:0000226; is a type of establishment of localization in cell [GO:0051649]; is a type of spindle localization [GO:0051653]; is a type of establishment of organelle localization [GO:0051656] Sources: GOC:ai Subtypes: establishment of mitotic spindle localization [GO:0040001], establishment of spindle orientation [GO:0051294], establishment of meiotic spindle localization [GO:0051295] Also known as: establishment of spindle localisation, spindle positioning